{
  "term_label": "regulation of cell migration",
  "term_id": "GO:0030334",
  "gene_symbol": "PLXNA2",
  "gene": "UniProtKB:O75051",
  "gene_name": "Plexin-A2"
}